cyclin D2-CDK4 complex [GO:0097129] (cellular component) Relationships: is a type of cyclin-dependent protein kinase holoenzyme complex [GO:0000307] References: PMID:15935619 Sources: GOC:so Definition: A protein complex consisting of cyclin D2 and cyclin-dependent kinase 4 (CDK4). Cyclins are characterized by periodicity in protein abundance throughout the cell cycle. Cyclin-dependent kinases represent a family of serine/threonine protein kinases that become active upon binding to a cyclin regulatory partner.